{
  "term_label": "osteoblast differentiation",
  "gene_symbol": "NOG",
  "term_id": "GO:0001649",
  "gene": "UniProtKB:Q13253",
  "gene_name": "Noggin"
}